{
  "gene_name": "Probable ATP-dependent RNA helicase DDX23",
  "term_id": "GO:0000398",
  "gene": "UniProtKB:Q9BUQ8",
  "gene_symbol": "DDX23",
  "term_label": "mRNA splicing, via spliceosome"
}